negative regulation of single-species biofilm formation on inanimate substrate [GO:1900232] (biological process) Also known as: down regulation of single-species biofilm formation on inanimate substrate, down-regulation of single-species biofilm formation on inanimate substrate, downregulation of single-species biofilm formation on inanimate substrate, inhibition of single-species biofilm formation on inanimate substrate Definition: Any process that stops, prevents or reduces the frequency, rate or extent of single-species biofilm formation on inanimate substrate. Sources: GOC:TermGenie, GOC:di Relationships: is a type of negative regulation of single-species biofilm formation [GO:1900191]; is_a GO:1900231; negatively regulates single-species biofilm formation on inanimate substrate [GO:0044011]